{
  "gene_symbol": "SEC16A",
  "gene": "UniProtKB:O15027",
  "term_label": "ER to Golgi transport vesicle membrane",
  "term_id": "GO:0012507",
  "gene_name": "Protein transport protein Sec16A"
}